{
  "gene_symbol": "BCL2L14",
  "term_label": "Unknown molecular function",
  "gene": "UniProtKB:Q9BZR8",
  "term_id": "UNKNOWN:0001",
  "gene_name": "Apoptosis facilitator Bcl-2-like protein 14"
}